{
  "term_label": "Unknown cellular component",
  "gene_symbol": "SPANXN3",
  "gene": "UniProtKB:Q5MJ09",
  "term_id": "UNKNOWN:0003",
  "gene_name": "Sperm protein associated with the nucleus on the X chromosome N3"
}